{
  "term_label": "N,N-dimethylaniline monooxygenase activity",
  "gene_name": "Flavin-containing monooxygenase 1",
  "gene": "UniProtKB:Q01740",
  "term_id": "GO:0004499",
  "gene_symbol": "FMO1"
}